{
  "gene_name": "Bone morphogenetic protein 6",
  "term_label": "extracellular space",
  "gene": "UniProtKB:P22004",
  "gene_symbol": "BMP6",
  "term_id": "GO:0005615"
}